mitochondrial L-ornithine transmembrane transport [GO:1990575] (biological process) References: PMID:9237680 Relationships: is a type of GO:1903352; is a type of mitochondrial transmembrane transport [GO:1990542] Definition: The process in which L-ornithine is transported across a mitochondrial membrane, into or out of the mitochondrion. Also known as: mitochondrial ornithine transmembrane transport, mitochondrial ornithine transport